{
  "term_label": "L-threonine transmembrane transporter activity",
  "gene_symbol": "SLC1A4",
  "gene_name": "Neutral amino acid transporter A",
  "term_id": "GO:0015195",
  "gene": "UniProtKB:P43007"
}